striated muscle adaptation [GO:0014888] (biological process) Definition: Any process in which striated muscle adapts, with consequent modifications to structural and/or functional phenotypes, in response to a stimulus. Stimuli include contractile activity, loading conditions, substrate supply, and environmental factors. These adaptive events occur in both muscle fibers and associated structures (motoneurons and capillaries), and they involve alterations in regulatory mechanisms, contractile properties and metabolic capacities. Sources: GOC:mtg_muscle Relationships: is a type of muscle adaptation [GO:0043500] Subtypes: cardiac muscle adaptation [GO:0014887], striated muscle atrophy [GO:0014891], skeletal muscle adaptation [GO:0043501] Also known as: striated muscle plasticity